{
  "gene": "UniProtKB:Q8N8E1",
  "gene_symbol": "MAPKAPK5-AS1",
  "term_label": "Unknown biological process",
  "gene_name": "Putative uncharacterized protein encoded by MAPKAPK5-AS1",
  "term_id": "UNKNOWN:0002"
}